{
  "term_id": "GO:0035556",
  "term_label": "intracellular signal transduction",
  "gene_symbol": "LRRC28",
  "gene": "UniProtKB:Q86X40",
  "gene_name": "Leucine-rich repeat-containing protein 28"
}